{
  "gene": "UniProtKB:Q92784",
  "gene_symbol": "DPF3",
  "term_id": "UNKNOWN:0001",
  "gene_name": "Zinc finger protein DPF3",
  "term_label": "Unknown molecular function"
}